neuropeptide receptor activity [GO:0008188] (molecular function) Relationships: is a type of G protein-coupled peptide receptor activity [GO:0008528]; is part of neuropeptide signaling pathway [GO:0007218]; has part neuropeptide binding [GO:0042923] Subtypes: neuromedin U receptor activity [GO:0001607], bombesin receptor activity [GO:0004946], galanin receptor activity [GO:0004966], corticotropin receptor activity [GO:0004978], beta-endorphin receptor activity [GO:0004979], GO:0004983, GO:0004994, GO:0004995, GO:0016492, GO:0035236, corazonin receptor activity [GO:0035237], L-DOPA receptor activity [GO:0035643], short neuropeptide F receptor activity [GO:0036400], pyrokinin receptor activity [GO:0036401], neuropeptide F receptor activity [GO:0042263] Definition: Combining with a neuropeptide to initiate a change in cell activity. Sources: GOC:ai